{
  "gene_name": "Zinc finger protein 30 homolog",
  "gene_symbol": "ZFP30",
  "term_id": "GO:0000978",
  "term_label": "RNA polymerase II cis-regulatory region sequence-specific DNA binding",
  "gene": "UniProtKB:Q9Y2G7"
}